{
  "gene": "UniProtKB:A0A075B6H8",
  "term_id": "GO:0019814",
  "term_label": "immunoglobulin complex",
  "gene_symbol": "IGKV1D-42",
  "gene_name": "Probable non-functional immunoglobulin kappa variable 1D-42"
}